{
  "gene": "UniProtKB:O75874",
  "gene_symbol": "IDH1",
  "gene_name": "Isocitrate dehydrogenase [NADP] cytoplasmic",
  "term_label": "cytosol",
  "term_id": "GO:0005829"
}